galactomannan binding [GO:2001072] (MF) Relationships: is_a heteropolysaccharide binding [GO:0010297] Definition: Binding to galactomannan. Sources: GOC:mengo_curators